{
  "gene_symbol": "FOXG1",
  "term_label": "sequence-specific double-stranded DNA binding",
  "term_id": "GO:1990837",
  "gene": "UniProtKB:P55316",
  "gene_name": "Forkhead box protein G1"
}